{
  "gene_symbol": "LYST",
  "term_label": "pigmentation",
  "term_id": "GO:0043473",
  "gene": "UniProtKB:Q99698",
  "gene_name": "Lysosomal-trafficking regulator"
}